{
  "gene_name": "Adenomatous polyposis coli protein",
  "term_label": "gamma-catenin binding",
  "term_id": "GO:0045295",
  "gene": "UniProtKB:P25054",
  "gene_symbol": "APC"
}